{
  "gene_name": "Olfactory receptor 3A3",
  "gene_symbol": "OR3A3",
  "gene": "UniProtKB:P47888",
  "term_id": "GO:0005886",
  "term_label": "plasma membrane"
}